{
  "term_label": "response to dsRNA",
  "gene": "UniProtKB:O15455",
  "term_id": "GO:0043331",
  "gene_name": "Toll-like receptor 3",
  "gene_symbol": "TLR3"
}